{
  "term_id": "GO:0030154",
  "gene_symbol": "NKX2-4",
  "gene_name": "Homeobox protein Nkx-2.4",
  "term_label": "cell differentiation",
  "gene": "UniProtKB:Q9H2Z4"
}